{
  "term_label": "positive regulation of angiogenesis",
  "term_id": "GO:0045766",
  "gene_name": "Endothelial transcription factor GATA-2",
  "gene": "UniProtKB:P23769",
  "gene_symbol": "GATA2"
}